renal vasodilation of the peripheral vascular system involved in regulation of systemic arterial blood pressure [GO:0003075] (biological process) Definition: The renal process that modulates the force with which blood travels through the circulatory system, by vasodilation of the peripheral vascular system. Sources: GOC:mtg_cardio Also known as: renal regulation of systemic arterial blood pressure by vasodilation of the peripheral vascular system Relationships: is a type of GO:0003072